{
  "term_id": "UNKNOWN:0002",
  "gene": "UniProtKB:Q6F5E7",
  "gene_symbol": "TXNRD3NB",
  "gene_name": "Putative uncharacterized protein TXNRD3NB",
  "term_label": "Unknown biological process"
}